{
  "gene_name": "Zinc finger CCHC domain-containing protein 14",
  "term_id": "UNKNOWN:0001",
  "gene": "UniProtKB:Q8WYQ9",
  "gene_symbol": "ZCCHC14",
  "term_label": "Unknown molecular function"
}